{
  "gene_symbol": "ORC6",
  "term_id": "UNKNOWN:0001",
  "gene_name": "Origin recognition complex subunit 6",
  "term_label": "Unknown molecular function",
  "gene": "UniProtKB:Q9Y5N6"
}